mannuronate reductase activity [GO:0050090] (molecular function) Definition: Catalysis of the reaction: D-mannonate + NAD(P)+ = D-mannuronate + NAD(P)H + H+. Also known as: D-mannonate:NAD(P)+ 6-oxidoreductase activity, D-mannonate:nicotinamide adenine dinucleotide (phosphate oxidoreductase (D-mannuronate-forming)), mannonate (nicotinamide adenine dinucleotide (phosphate))dehydrogenase activity, mannonate dehydrogenase (NAD(P)+), mannonate dehydrogenase activity Relationships: is a type of oxidoreductase activity, acting on the CH-OH group of donors, NAD or NADP as acceptor [GO:0016616] Sources: EC:1.1.1.131, MetaCyc:MANNURONATE-REDUCTASE-RXN